{
  "term_label": "immune response-inhibiting cell surface receptor signaling pathway",
  "gene_symbol": "LILRA5",
  "gene_name": "Leukocyte immunoglobulin-like receptor subfamily A member 5",
  "term_id": "GO:0002767",
  "gene": "UniProtKB:A6NI73"
}